DNA gyrase complex [GO:0120217] (cellular component) Definition: A bacterial type IIA topoisomerase that is unique in its function of introducing negative supercoils into DNA at the expense of ATP hydrolysis and is also capable of relaxing positive supercoils, an activity shared with topoisomerase IV. Typically, it is composed of two copies each of an A subunit (GyrA) and a B subunit (GyrB). References: PMID:1657531, PMID:20675723 Sources: GOC:bhm, GOC:krc, Wikipedia:DNA_gyrase Also known as: topoisomerase II complex Relationships: is a type of DNA topoisomerase type II (double strand cut, ATP-hydrolyzing) complex [GO:0009330]